{
  "term_label": "cytoplasm",
  "term_id": "GO:0005737",
  "gene": "UniProtKB:Q9Y5S2",
  "gene_symbol": "CDC42BPB",
  "gene_name": "Serine_threonine-protein kinase MRCK beta"
}